{
  "term_id": "GO:0003713",
  "gene_symbol": "KMT2C",
  "gene_name": "Histone-lysine N-methyltransferase 2C",
  "term_label": "transcription coactivator activity",
  "gene": "UniProtKB:Q8NEZ4"
}